{
  "gene": "UniProtKB:P19013",
  "gene_symbol": "KRT4",
  "gene_name": "Keratin, type II cytoskeletal 4",
  "term_id": "GO:0031424",
  "term_label": "keratinization"
}